{
  "gene": "UniProtKB:Q8NGH5",
  "term_label": "Unknown biological process",
  "gene_symbol": "OR56A1",
  "term_id": "UNKNOWN:0002",
  "gene_name": "Olfactory receptor 56A1"
}